{
  "gene": "UniProtKB:Q9UNK0",
  "term_id": "GO:0006886",
  "gene_symbol": "STX8",
  "term_label": "intracellular protein transport",
  "gene_name": "Syntaxin-8"
}